{
  "gene": "UniProtKB:O95760",
  "gene_name": "Interleukin-33",
  "gene_symbol": "IL33",
  "term_label": "positive regulation of inflammatory response",
  "term_id": "GO:0050729"
}